{
  "term_id": "UNKNOWN:0003",
  "gene_symbol": "FHIP2B",
  "gene_name": "FHF complex subunit HOOK-interacting protein 2B",
  "gene": "UniProtKB:Q86V87",
  "term_label": "Unknown cellular component"
}